{
  "term_label": "tRNA processing",
  "gene_name": "Lupus La protein",
  "term_id": "GO:0008033",
  "gene": "UniProtKB:P05455",
  "gene_symbol": "SSB"
}